{
  "gene_name": "Zinc finger protein 263",
  "term_label": "regulation of transcription by RNA polymerase II",
  "gene": "UniProtKB:O14978",
  "gene_symbol": "ZNF263",
  "term_id": "GO:0006357"
}